corticotropin-releasing hormone activity [GO:0017045] (molecular function) Definition: The action characteristic of corticotropin-releasing hormone (CRH), any of a number of peptides released by the mammalian hypothalamus into the hypophyseal-portal circulation in response to neural and/or chemical stimuli. Upon receptor binding, CRH increases the rate of corticotropin secretion by the anterior pituitary. Relationships: is a type of hormone activity [GO:0005179] Sources: ISBN:0198506732 Also known as: adrenocorticotropin-releasing hormone